{
  "gene": "UniProtKB:Q6ZUT6",
  "gene_symbol": "CCDC9B",
  "term_id": "UNKNOWN:0001",
  "gene_name": "Coiled-coil domain-containing protein 9B",
  "term_label": "Unknown molecular function"
}